{
  "gene": "UniProtKB:Q9ULE0",
  "gene_symbol": "WWC3",
  "gene_name": "Protein WWC3",
  "term_label": "cytoplasm",
  "term_id": "GO:0005737"
}